{
  "gene": "UniProtKB:Q8NGI1",
  "term_label": "olfactory receptor activity",
  "gene_symbol": "OR56B2",
  "gene_name": "Putative olfactory receptor 56B2",
  "term_id": "GO:0004984"
}